CLRC complex localization to heterochromatin [GO:0044382] (biological process) Sources: GOC:jl Also known as: CLRC ubiquitin ligase complex localisation to heterochromatin, CLRC ubiquitin ligase complex localization to heterochromatin Relationships: is a type of protein-containing complex localization [GO:0031503]; is a type of protein localization to heterochromatin [GO:0097355] Definition: The process by which a CLRC complex is transported to, or maintained in, heterochromatin. CLRC complex is an active cullin-dependent E3 ubiquitin ligase complex essential for heterochromatin assembly by RNAi and histone H3K9 methylation.